histone isonicotinyltransferase activity [GO:0140230] (MF) References: PMID:34545082 Definition: Catalysis of the reaction: isonicotinyl-CoA + histone = coA + N(6)-isonicotinyl-histone. Relationships: is a type of histone modifying activity [GO:0140993]